phosphatidylinositol 3-kinase regulator activity [GO:0035014] (MF) Definition: Modulates the activity of a phosphatidylinositol 3-kinase (PI3K). Regulatory subunits can link a PI3K catalytic subunit to upstream signaling events and help position the catalytic subunits close to their lipid substrates. References: PMID:9255069 Sources: GOC:bf Also known as: PI3K regulator activity, phosphoinositide 3-kinase regulator activity Note: See also the molecular function term 'phosphoinositide 3-kinase activity ; GO:0035004'. Relationships: is a type of kinase regulator activity [GO:0019207]; BFO_0000051 GO:0036313 Subtypes: phosphatidylinositol 3-kinase activator activity [GO:0141038], phosphatidylinositol 3-kinase inhibitor activity [GO:0141039]